anal fin development [GO:0033335] (biological process) Definition: The process whose specific outcome is the progression of the anal fin over time, from its formation to the mature structure. Sources: GOC:dgh Relationships: is a type of GO:0033338